{
  "term_label": "stem cell population maintenance",
  "gene": "UniProtKB:Q8N7R0",
  "gene_name": "Putative homeobox protein NANOG2",
  "gene_symbol": "NANOGP1",
  "term_id": "GO:0019827"
}